{
  "gene_name": "Dynamin-3",
  "gene_symbol": "DNM3",
  "term_label": "microtubule",
  "term_id": "GO:0005874",
  "gene": "UniProtKB:Q9UQ16"
}